positive regulation of the force of heart contraction by epinephrine [GO:0003059] (biological process) Relationships: is_a positive regulation of the force of heart contraction by chemical signal [GO:0003099]; is part of positive regulation of the force of heart contraction by epinephrine-norepinephrine [GO:0001997] Definition: The process in which the secretion of epinephrine into the bloodstream or released from nerve endings modulates the force of heart muscle contraction. Subtypes: positive regulation of the force of heart contraction by neuronal epinephrine [GO:0003087], positive regulation of the force of heart contraction by circulating epinephrine [GO:0003088] Also known as: adrenaline cardiac inotropy, adrenaline regulation of the strength of heart muscle contraction, epinephrine cardiac inotropy, increased force of heart contraction by epinephrine, positive regulation of heart contraction by adrenaline, positive regulation of heart contraction by epinephrine Sources: GOC:mtg_cardio, GOC:rl